{
  "term_id": "GO:0030027",
  "gene_name": "Actin-binding protein WASF2",
  "gene_symbol": "WASF2",
  "term_label": "lamellipodium",
  "gene": "UniProtKB:Q9Y6W5"
}